{
  "term_id": "GO:0000977",
  "gene_symbol": "ZBTB46",
  "term_label": "RNA polymerase II transcription regulatory region sequence-specific DNA binding",
  "gene_name": "Zinc finger and BTB domain-containing protein 46",
  "gene": "UniProtKB:Q86UZ6"
}